{
  "gene_symbol": "AGBL4",
  "gene": "UniProtKB:Q5VU57",
  "term_label": "ciliary basal body",
  "gene_name": "Cytosolic carboxypeptidase 6",
  "term_id": "GO:0036064"
}